{
  "gene_name": "Zinc finger protein PLAG1",
  "term_label": "regulation of DNA-templated transcription",
  "term_id": "GO:0006355",
  "gene": "UniProtKB:Q6DJT9",
  "gene_symbol": "PLAG1"
}